{
  "gene": "UniProtKB:Q15617",
  "term_label": "sensory perception of smell",
  "term_id": "GO:0007608",
  "gene_symbol": "OR8G1",
  "gene_name": "Olfactory receptor 8G1"
}